{
  "gene": "UniProtKB:Q9UPN4",
  "term_id": "GO:0010824",
  "gene_symbol": "CEP131",
  "term_label": "regulation of centrosome duplication",
  "gene_name": "Centrosomal protein of 131 kDa"
}